negative regulation of guanylate cyclase activity [GO:0031283] (biological process) Definition: Any process that stops, prevents, or reduces the frequency, rate or extent of guanylate cyclase activity. Relationships: is a type of GO:0043086; is a type of GO:1900372; negatively regulates GO:0004383 Also known as: down regulation of guanylate cyclase activity, down-regulation of guanylate cyclase activity, downregulation of guanylate cyclase activity, inhibition of guanylate cyclase activity Sources: GOC:mah